regulation of apoptotic process involved in development [GO:1904748] (biological process) Subtypes: regulation of B cell deletion [GO:0002867], regulation of nurse cell apoptotic process [GO:0045477], regulation of mesenchymal cell apoptotic process involved in metanephros development [GO:1900211], regulation of apoptotic process involved in metanephric collecting duct development [GO:1900214], GO:1900217, regulation of apoptotic process involved in morphogenesis [GO:1902337], GO:1904746, GO:1904747 References: PMID:22801495 Sources: GOC:TermGenie, GO_REF:0000058 Definition: Any process that modulates the frequency, rate or extent of apoptotic process involved in development. Relationships: is a type of regulation of apoptotic process [GO:0042981]; is a type of GO:0050793; regulates apoptotic process involved in development [GO:1902742] Note: Q10943 in PMID:22801495, inferred from mutant phenotype Also known as: regulation of apoptotic cell death involved in anatomical structure development, regulation of apoptotic cell death involved in development of an anatomical structure, regulation of apoptotic process involved in anatomical structure development, regulation of apoptotic process involved in development of an anatomical structure, regulation of apoptotic programmed cell death involved in anatomical structure development, regulation of apoptotic programmed cell death involved in development of an anatomical structure, regulation of programmed cell death by apoptosis involved in anatomical structure development, regulation of programmed cell death by apoptosis involved in development of an anatomical structure, regulation of activation of apoptosis involved in anatomical structure development, regulation of activation of apoptosis involved in development of an anatomical structure, regulation of apoptosis involved in anatomical structure development, regulation of apoptosis involved in development of an anatomical structure, regulation of apoptosis signaling involved in anatomical structure development, regulation of apoptosis signaling involved in development of an anatomical structure, regulation of apoptotic program involved in anatomical structure development, regulation of apoptotic program involved in development of an anatomical structure, regulation of type I programmed cell death involved in anatomical structure development, regulation of type I programmed cell death involved in development of an anatomical structure, regulation of apoptosis activator activity involved in anatomical structure development, regulation of apoptosis activator activity involved in development of an anatomical structure, regulation of commitment to apoptosis involved in anatomical structure development, regulation of commitment to apoptosis involved in development of an anatomical structure, regulation of induction of apoptosis by p53 involved in anatomical structure development, regulation of induction of apoptosis by p53 involved in development of an anatomical structure, regulation of induction of apoptosis involved in anatomical structure development, regulation of induction of apoptosis involved in development of an anatomical structure, regulation of signaling (initiator) caspase activity involved in anatomical structure development, regulation of signaling (initiator) caspase activity involved in development of an anatomical structure